{
  "term_label": "RNA helicase activity",
  "gene": "UniProtKB:Q7L2E3",
  "gene_name": "ATP-dependent RNA helicase DHX30",
  "term_id": "GO:0003724",
  "gene_symbol": "DHX30"
}